{
  "gene": "UniProtKB:Q8TEK3",
  "term_label": "DNA repair",
  "gene_symbol": "DOT1L",
  "term_id": "GO:0006281",
  "gene_name": "Histone-lysine N-methyltransferase, H3 lysine-79 specific"
}